SCF-Grr1/Pof2 ubiquitin ligase complex [GO:0097664] (cellular component) Relationships: is a type of SCF ubiquitin ligase complex [GO:0019005] References: PMID:10213692, PMID:15147268 Sources: GOC:jd, GOC:vw Definition: An SCF ubiquitin ligase complex in which the F-box protein is Grr1 in S. cerevisiae (Pof2 in S. pombe).